{
  "term_label": "adherens junction",
  "gene": "UniProtKB:P12830",
  "gene_symbol": "CDH1",
  "gene_name": "Cadherin-1",
  "term_id": "GO:0005912"
}